{
  "term_id": "GO:0038003",
  "gene_name": "Delta-type opioid receptor",
  "term_label": "G protein-coupled opioid receptor signaling pathway",
  "gene": "UniProtKB:P41143",
  "gene_symbol": "OPRD1"
}